{
  "term_id": "UNKNOWN:0002",
  "gene_name": "Late cornified envelope protein 7A",
  "term_label": "Unknown biological process",
  "gene": "UniProtKB:P0DV60",
  "gene_symbol": "LCE7A"
}